{
  "term_id": "GO:0005634",
  "gene_name": "Mitogen-activated protein kinase 4",
  "term_label": "nucleus",
  "gene": "UniProtKB:P31152",
  "gene_symbol": "MAPK4"
}